{
  "gene": "UniProtKB:P62280",
  "term_label": "structural constituent of ribosome",
  "gene_name": "Small ribosomal subunit protein uS17",
  "gene_symbol": "RPS11",
  "term_id": "GO:0003735"
}